symbiont-mediated suppression of host pathogen-associated molecular pattern receptor signaling pathway [GO:0052078] (biological process) Definition: A process in which a symbiont interferes with, inhibits or disrupts a PAMP signaling pathway in its host organism, initiated by a ligand binding of a pattern recognition receptor (PRR) to activate a plant innate immune response. The host is defined as the larger of the organisms involved in a symbiotic interaction. References: PMID:18005697 Also known as: disruption of host PAMP receptor signaling pathway, disruption of host pathogen-associated molecular pattern receptor signaling pathway, suppression of host pathogen-associated molecular pattern receptor signaling pathway Relationships: is_a symbiont-mediated suppression of host signal transduction pathway [GO:0052029]; is a type of symbiont-mediated suppression of host innate immune response [GO:0052170] Subtypes: symbiont-mediated suppression of cytoplasmic pattern recognition receptor signaling pathway [GO:0039537]